{
  "gene_name": "Dehydrogenase_reductase SDR family member 12",
  "term_id": "UNKNOWN:0003",
  "term_label": "Unknown cellular component",
  "gene_symbol": "DHRS12",
  "gene": "UniProtKB:A0PJE2"
}